guanosine tetraphosphate binding [GO:0097216] (molecular function) References: PMID:15109491, PMID:16968770, PMID:18359660 Sources: GOC:imk Also known as: 5'-ppGpp-3' binding Definition: Binding to guanosine tetraphosphate (5'-ppGpp-3'), a guanosine bisphosphate having diphosphate groups at both the 3' and 5'-positions. Relationships: is a type of guanyl ribonucleotide binding [GO:0032561]; is a type of anion binding [GO:0043168]